{
  "gene_symbol": "MAGI2",
  "term_id": "GO:0046332",
  "gene_name": "Membrane-associated guanylate kinase, WW and PDZ domain-containing protein 2",
  "term_label": "SMAD binding",
  "gene": "UniProtKB:Q86UL8"
}